{
  "term_id": "GO:0016081",
  "term_label": "synaptic vesicle docking",
  "gene_name": "Protein unc-13 homolog B",
  "gene_symbol": "UNC13B",
  "gene": "UniProtKB:O14795"
}